sphingolipid transporter activity [GO:0046624] (molecular function) Subtypes: sphingolipid floppase activity [GO:0046623], GO:0120016, glycosylceramide flippase activity [GO:0140351] Relationships: is a type of lipid transporter activity [GO:0005319] Definition: Enables the directed movement of sphingolipids into, out of or within a cell, or between cells. Sphingolipids are a class of lipids containing the long-chain amine diol sphingosine or a closely related base (a sphingoid). Sources: GOC:ai, ISBN:0198506732